gliotoxin biosynthetic process [GO:2001310] (biological process) Definition: The chemical reactions and pathways resulting in the formation of the epipolythiodioxopiperazine gliotoxin, a poisonous substance produced by some species of fungi. Regulation: regulated by regulation of gliotoxin biosynthetic process [GO:1900689]; negatively regulated by negative regulation of gliotoxin biosynthetic process [GO:1900690]; positively regulated by positive regulation of gliotoxin biosynthetic process [GO:1900691] References: PMID:16333108, PMID:17574915, PMID:18272357, PMID:29966253 Sources: GOC:di Relationships: is a type of GO:0043386; is a type of amide biosynthetic process [GO:0043604]; is a type of sulfur compound biosynthetic process [GO:0044272]; has part gamma-glutamylcyclotransferase activity [GO:0003839]; has part GO:0004364; has part monooxygenase activity [GO:0004497]; has part N-methyltransferase activity [GO:0008170]; has part transaminase activity [GO:0008483]; has part disulfide oxidoreductase activity [GO:0015036]; has part acid-amino acid ligase activity [GO:0016881] Also known as: gliotoxin anabolism, gliotoxin biosynthesis, gliotoxin formation, gliotoxin synthesis